{
  "term_label": "membrane",
  "gene_symbol": "SLC45A4",
  "gene_name": "Solute carrier family 45 member 4",
  "term_id": "GO:0016020",
  "gene": "UniProtKB:Q5BKX6"
}